{
  "gene_name": "Zinc finger protein 425",
  "term_id": "GO:0000977",
  "gene": "UniProtKB:Q6IV72",
  "gene_symbol": "ZNF425",
  "term_label": "RNA polymerase II transcription regulatory region sequence-specific DNA binding"
}